{
  "gene_symbol": "MYO15A",
  "term_id": "GO:0016020",
  "gene_name": "Unconventional myosin-XV",
  "gene": "UniProtKB:Q9UKN7",
  "term_label": "membrane"
}